{
  "term_label": "phospholipase C-activating G protein-coupled receptor signaling pathway",
  "gene_symbol": "P2RY1",
  "gene": "UniProtKB:P47900",
  "gene_name": "P2Y purinoceptor 1",
  "term_id": "GO:0007200"
}